{
  "gene": "UniProtKB:Q9P2F6",
  "gene_name": "Rho GTPase-activating protein 20",
  "term_label": "Unknown biological process",
  "term_id": "UNKNOWN:0002",
  "gene_symbol": "ARHGAP20"
}